negative regulation of kojic acid biosynthetic process [GO:1900395] (BP) Also known as: down regulation of 5-hydroxy-2-(hydroxymethyl)-4H-pyran-4-one anabolism, down regulation of 5-hydroxy-2-(hydroxymethyl)-4H-pyran-4-one biosynthesis, down regulation of 5-hydroxy-2-(hydroxymethyl)-4H-pyran-4-one biosynthetic process, down regulation of 5-hydroxy-2-(hydroxymethyl)-4H-pyran-4-one formation, down regulation of 5-hydroxy-2-(hydroxymethyl)-4H-pyran-4-one synthesis, down regulation of kojic acid anabolism, down regulation of kojic acid biosynthesis, down regulation of kojic acid biosynthetic process, down regulation of kojic acid formation, down regulation of kojic acid synthesis, down-regulation of 5-hydroxy-2-(hydroxymethyl)-4H-pyran-4-one anabolism, down-regulation of 5-hydroxy-2-(hydroxymethyl)-4H-pyran-4-one biosynthesis, down-regulation of 5-hydroxy-2-(hydroxymethyl)-4H-pyran-4-one biosynthetic process, down-regulation of 5-hydroxy-2-(hydroxymethyl)-4H-pyran-4-one formation, down-regulation of 5-hydroxy-2-(hydroxymethyl)-4H-pyran-4-one synthesis, down-regulation of kojic acid anabolism, down-regulation of kojic acid biosynthesis, down-regulation of kojic acid biosynthetic process, down-regulation of kojic acid formation, down-regulation of kojic acid synthesis, downregulation of 5-hydroxy-2-(hydroxymethyl)-4H-pyran-4-one anabolism, downregulation of 5-hydroxy-2-(hydroxymethyl)-4H-pyran-4-one biosynthesis, downregulation of 5-hydroxy-2-(hydroxymethyl)-4H-pyran-4-one biosynthetic process, downregulation of 5-hydroxy-2-(hydroxymethyl)-4H-pyran-4-one formation, downregulation of 5-hydroxy-2-(hydroxymethyl)-4H-pyran-4-one synthesis, downregulation of kojic acid anabolism, downregulation of kojic acid biosynthesis, downregulation of kojic acid biosynthetic process, downregulation of kojic acid formation, downregulation of kojic acid synthesis, inhibition of 5-hydroxy-2-(hydroxymethyl)-4H-pyran-4-one anabolism, inhibition of 5-hydroxy-2-(hydroxymethyl)-4H-pyran-4-one biosynthesis, inhibition of 5-hydroxy-2-(hydroxymethyl)-4H-pyran-4-one biosynthetic process, inhibition of 5-hydroxy-2-(hydroxymethyl)-4H-pyran-4-one formation, inhibition of 5-hydroxy-2-(hydroxymethyl)-4H-pyran-4-one synthesis, inhibition of kojic acid anabolism, inhibition of kojic acid biosynthesis, inhibition of kojic acid formation, inhibition of kojic acid synthesis, negative regulation of 5-hydroxy-2-(hydroxymethyl)-4H-pyran-4-one anabolism, negative regulation of 5-hydroxy-2-(hydroxymethyl)-4H-pyran-4-one biosynthesis, negative regulation of 5-hydroxy-2-(hydroxymethyl)-4H-pyran-4-one biosynthetic process, negative regulation of 5-hydroxy-2-(hydroxymethyl)-4H-pyran-4-one formation, negative regulation of 5-hydroxy-2-(hydroxymethyl)-4H-pyran-4-one synthesis, negative regulation of kojic acid anabolism, negative regulation of kojic acid biosynthesis, negative regulation of kojic acid formation, negative regulation of kojic acid synthesis, inhibition of kojic acid biosynthetic process, down regulation of C6H6O4 anabolism, down regulation of C6H6O4 biosynthesis, down regulation of C6H6O4 biosynthetic process, down regulation of C6H6O4 formation, down regulation of C6H6O4 synthesis, down-regulation of C6H6O4 anabolism, down-regulation of C6H6O4 biosynthesis, down-regulation of C6H6O4 biosynthetic process, down-regulation of C6H6O4 formation, down-regulation of C6H6O4 synthesis, downregulation of C6H6O4 anabolism, downregulation of C6H6O4 biosynthesis, downregulation of C6H6O4 biosynthetic process, downregulation of C6H6O4 formation, downregulation of C6H6O4 synthesis, inhibition of C6H6O4 anabolism, inhibition of C6H6O4 biosynthesis, inhibition of C6H6O4 biosynthetic process, inhibition of C6H6O4 formation, inhibition of C6H6O4 synthesis, negative regulation of C6H6O4 anabolism, negative regulation of C6H6O4 biosynthesis, negative regulation of C6H6O4 biosynthetic process, negative regulation of C6H6O4 formation, negative regulation of C6H6O4 synthesis Sources: GOC:TermGenie, GOC:di Relationships: is a type of regulation of kojic acid biosynthetic process [GO:1900394]; is a type of negative regulation of alcohol biosynthetic process [GO:1902931]; RO_0002212 GO:2001317 Definition: Any process that stops, prevents or reduces the frequency, rate or extent of kojic acid biosynthetic process.